{
  "gene_name": "Polycomb group RING finger protein 2",
  "term_id": "GO:0000122",
  "gene": "UniProtKB:P35227",
  "gene_symbol": "PCGF2",
  "term_label": "negative regulation of transcription by RNA polymerase II"
}